{
  "term_id": "GO:0098887",
  "gene_name": "Ras-related protein Rab-11A",
  "gene": "UniProtKB:P62491",
  "gene_symbol": "RAB11A",
  "term_label": "neurotransmitter receptor transport, endosome to postsynaptic membrane"
}